{
  "gene_symbol": "PEX14",
  "term_label": "peroxisomal membrane",
  "gene": "UniProtKB:O75381",
  "term_id": "GO:0005778",
  "gene_name": "Peroxisomal membrane protein PEX14"
}